serine-type exopeptidase activity [GO:0070008] (molecular function) Sources: GOC:mah, https://www.ebi.ac.uk/merops/about/glossary.shtml#CATTYPE, https://www.ebi.ac.uk/merops/about/glossary.shtml#EXOPEPTIDASE Definition: Catalysis of the hydrolysis of a peptide bond not more than three residues from the N- or C-terminus of a polypeptide chain by a catalytic mechanism that involves a catalytic triad consisting of a serine nucleophile that is activated by a proton relay involving an acidic residue (e.g. aspartate or glutamate) and a basic residue (usually histidine). Relationships: is a type of serine-type peptidase activity [GO:0008236]; is_a exopeptidase activity [GO:0008238] Subtypes: serine-type carboxypeptidase activity [GO:0004185], tripeptidyl-peptidase activity [GO:0008240], serine-type aminopeptidase activity [GO:0070009]